{
  "gene_symbol": "SEMA4G",
  "term_id": "GO:0038191",
  "term_label": "neuropilin binding",
  "gene_name": "Semaphorin-4G",
  "gene": "UniProtKB:Q9NTN9"
}